{
  "term_label": "fibroblast growth factor binding",
  "gene": "UniProtKB:P35052",
  "gene_name": "Glypican-1",
  "gene_symbol": "GPC1",
  "term_id": "GO:0017134"
}